somite specification [GO:0001757] (biological process) Relationships: is a type of segment specification [GO:0007379]; is a type of GO:0009880; BFO_0000050 somitogenesis [GO:0001756] Sources: GOC:dph Definition: The process in which individual somites establish identity during embryogenesis.